{
  "gene_name": "Muscarinic acetylcholine receptor M4",
  "term_label": "chemical synaptic transmission",
  "gene": "UniProtKB:P08173",
  "gene_symbol": "CHRM4",
  "term_id": "GO:0007268"
}